{
  "gene": "UniProtKB:P27338",
  "term_label": "mitochondrion",
  "gene_name": "Amine oxidase [flavin-containing] B",
  "term_id": "GO:0005739",
  "gene_symbol": "MAOB"
}